{
  "term_id": "UNKNOWN:0003",
  "gene": "UniProtKB:P0DV60",
  "gene_name": "Late cornified envelope protein 7A",
  "term_label": "Unknown cellular component",
  "gene_symbol": "LCE7A"
}